negative regulation of plasma membrane repair [GO:1905685] (biological process) Definition: Any process that stops, prevents or reduces the frequency, rate or extent of plasma membrane repair. Also known as: down regulation of plasma membrane repair, down-regulation of plasma membrane repair, downregulation of plasma membrane repair, inhibition of plasma membrane repair Relationships: is a type of negative regulation of cellular component organization [GO:0051129]; is a type of negative regulation of wound healing [GO:0061045]; is a type of regulation of plasma membrane repair [GO:1905684]; negatively regulates GO:0001778 References: PMID:22940583 Sources: GOC:TermGenie, GOC:bhm, GO_REF:0000058